maintenance of protein localization at growing cell tip [GO:0099019] (biological process) Relationships: is a type of maintenance of protein localization at cell tip [GO:0099017]; BFO_0000066 growing cell tip [GO:0035838] Also known as: maintenance of protein location at growing cell tip References: PMID:24146635 Sources: GOC:dos, GOC:vw Definition: Any process in which localization of a protein is maintained at the growing cell tip.